inositol-3,4,5,6-tetrakisphosphate 1-kinase activity [GO:0047325] (molecular function) Also known as: inositol tetrakisphosphate 1-kinase activity, inositol 3,4,5,6-tetrakisphosphate 1-kinase activity, 1D-myo-inositol-tetrakisphosphate 1-kinase activity, 1D-myo-inositol-trisphosphate 5-kinase activity, 1D-myo-inositol-trisphosphate 6-kinase activity, ATP:1D-myo-inositol-3,4,5,6-tetrakisphosphate 1-phosphotransferase activity, inositol-trisphosphate 5-kinase activity, inositol-trisphosphate 6-kinase activity Sources: RHEA:12452 Relationships: is a type of inositol tetrakisphosphate kinase activity [GO:0051765] Definition: Catalysis of the reaction: 1D-myo-inositol 3,4,5,6-tetrakisphosphate + ATP = 1D-myo-inositol 1,3,4,5,6-pentakisphosphate + ADP + H+.